regulation of response to butan-1-ol [GO:1901448] (biological process) Relationships: is a type of GO:1901419; regulates GO:1901422 Subtypes: negative regulation of response to butan-1-ol [GO:1901449], positive regulation of response to butan-1-ol [GO:1901450] Sources: GOC:TermGenie, GOC:mengo_curators Definition: Any process that modulates the frequency, rate or extent of response to butan-1-ol.